{
  "gene_name": "rRNA methyltransferase 2, mitochondrial",
  "term_id": "GO:0008650",
  "gene": "UniProtKB:Q9UI43",
  "gene_symbol": "MRM2",
  "term_label": "rRNA (uridine-2'-O-)-methyltransferase activity"
}